regulation of receptor catabolic process [GO:2000644] (biological process) Relationships: is a type of regulation of catabolic process [GO:0009894]; is a type of regulation of macromolecule metabolic process [GO:0060255]; regulates receptor catabolic process [GO:0032801] Definition: Any process that modulates the frequency, rate or extent of receptor catabolic process. Subtypes: GO:0032803, negative regulation of receptor catabolic process [GO:2000645], positive regulation of receptor catabolic process [GO:2000646] Also known as: regulation of receptor breakdown, regulation of receptor catabolism, regulation of receptor degradation Sources: GOC:BHF